methylcrotonoyl-CoA carboxylase complex [GO:1905202] (cellular component) Relationships: is a type of catalytic complex [GO:1902494] Definition: A protein complex capable of methylcrotonoyl-CoA carboxylase activity. In mammals, it is a mitochondrial complex comprising a dodecamer of 6 alpha and 6 beta subunits: MCCC-alpha has a covalently bound biotin essential for the ATP-dependent carboxylation; MCCC-beta possesses carboxyltransferase activity which presumably is essential for binding to 3-methylcrotonyl-CoA. References: PMID:15868465, PMID:17360195, PMID:22158123, PMID:22869039 Sources: GOC:PARL, GOC:bf, GOC:hjd